{
  "gene_symbol": "ACKR3",
  "term_label": "external side of plasma membrane",
  "gene_name": "Atypical chemokine receptor 3",
  "gene": "UniProtKB:P25106",
  "term_id": "GO:0009897"
}